positive regulation of programmed necrotic cell death [GO:0062100] (biological process) Relationships: is a type of GO:0043068; is a type of regulation of programmed necrotic cell death [GO:0062098]; positively regulates programmed necrotic cell death [GO:0097300] References: PMID:27258785 Sources: GOC:aruk, GOC:rph Subtypes: positive regulation of necroptotic process [GO:0060545] Definition: Any process that increases the frequency, rate or extent of programmed necrotic cell death.